{
  "gene_symbol": "MAP9",
  "gene_name": "Microtubule-associated protein 9",
  "gene": "UniProtKB:Q49MG5",
  "term_id": "GO:0008017",
  "term_label": "microtubule binding"
}